{
  "term_id": "GO:0005654",
  "gene_symbol": "MIER3",
  "gene_name": "Mesoderm induction early response protein 3",
  "term_label": "nucleoplasm",
  "gene": "UniProtKB:Q7Z3K6"
}